{
  "term_id": "GO:0008277",
  "gene_name": "ARF GTPase-activating protein GIT2",
  "gene_symbol": "GIT2",
  "gene": "UniProtKB:Q14161",
  "term_label": "regulation of G protein-coupled receptor signaling pathway"
}